negative regulation of smooth muscle tissue development [GO:1905900] (biological process) Relationships: is a type of negative regulation of muscle tissue development [GO:1901862]; is a type of regulation of smooth muscle tissue development [GO:1905899]; negatively regulates smooth muscle tissue development [GO:0048745] Also known as: down regulation of smooth muscle tissue development, down-regulation of smooth muscle tissue development, downregulation of smooth muscle tissue development, inhibition of smooth muscle tissue development Definition: Any process that stops, prevents or reduces the frequency, rate or extent of smooth muscle tissue development. References: PMID:14709716 Sources: GOC:TermGenie, GOC:bhm, GO_REF:0000058